{
  "term_label": "tRNA wobble position uridine thiolation",
  "gene_name": "Adenylyltransferase and sulfurtransferase MOCS3",
  "term_id": "GO:0002143",
  "gene_symbol": "MOCS3",
  "gene": "UniProtKB:O95396"
}